{
  "term_id": "GO:0070098",
  "gene_symbol": "CCL4L1",
  "gene": "UniProtKB:Q8NHW4",
  "gene_name": "C-C motif chemokine 4-like",
  "term_label": "chemokine-mediated signaling pathway"
}